{
  "term_label": "Unknown cellular component",
  "gene": "UniProtKB:P04062",
  "gene_name": "Lysosomal acid glucosylceramidase",
  "gene_symbol": "GBA1",
  "term_id": "UNKNOWN:0003"
}